{
  "term_label": "axon guidance",
  "gene_symbol": "SEMA4G",
  "gene": "UniProtKB:Q9NTN9",
  "term_id": "GO:0007411",
  "gene_name": "Semaphorin-4G"
}